{
  "gene": "UniProtKB:O75368",
  "gene_name": "Adapter SH3BGRL",
  "term_id": "GO:1990756",
  "term_label": "ubiquitin-like ligase-substrate adaptor activity",
  "gene_symbol": "SH3BGRL"
}